{
  "gene": "UniProtKB:Q8N139",
  "gene_symbol": "ABCA6",
  "term_label": "lipid transport",
  "term_id": "GO:0006869",
  "gene_name": "ATP-binding cassette sub-family A member 6"
}